{
  "gene": "UniProtKB:Q9BSJ2",
  "gene_name": "Gamma-tubulin complex component 2",
  "term_label": "gamma-tubulin binding",
  "term_id": "GO:0043015",
  "gene_symbol": "TUBGCP2"
}